{
  "term_id": "GO:0003729",
  "gene_name": "Protein KHNYN",
  "gene_symbol": "KHNYN",
  "term_label": "mRNA binding",
  "gene": "UniProtKB:O15037"
}